negative regulation of mononuclear cell proliferation [GO:0032945] (biological process) Definition: Any process that stops, prevents, or reduces the frequency, rate or extent of mononuclear cell proliferation. Sources: GOC:add Also known as: negative regulation of PBMC proliferation, negative regulation of peripheral blood mononuclear cell proliferation Relationships: is a type of GO:0032944; is a type of GO:0070664; RO_0002212 mononuclear cell proliferation [GO:0032943] Subtypes: negative regulation of lymphocyte proliferation [GO:0050672]